{
  "term_id": "UNKNOWN:0003",
  "gene": "UniProtKB:Q13395",
  "gene_symbol": "TARBP1",
  "gene_name": "Probable methyltransferase TARBP1",
  "term_label": "Unknown cellular component"
}